{
  "gene": "UniProtKB:O15467",
  "gene_symbol": "CCL16",
  "gene_name": "C-C motif chemokine 16",
  "term_id": "GO:0006954",
  "term_label": "inflammatory response"
}